{
  "gene": "UniProtKB:P15538",
  "gene_symbol": "CYP11B1",
  "term_id": "GO:0032342",
  "gene_name": "Cytochrome P450 11B1, mitochondrial",
  "term_label": "aldosterone biosynthetic process"
}